{
  "gene_name": "Ubiquilin-1",
  "gene_symbol": "UBQLN1",
  "term_label": "autophagosome",
  "term_id": "GO:0005776",
  "gene": "UniProtKB:Q9UMX0"
}